{
  "gene_name": "Fibroblast growth factor receptor 2",
  "gene_symbol": "FGFR2",
  "gene": "UniProtKB:P21802",
  "term_label": "positive regulation of MAPK cascade",
  "term_id": "GO:0043410"
}